neural tube development [GO:0021915] (biological process) Relationships: is a type of GO:0035295; is a type of GO:0060429; is part of GO:0007399; is part of chordate embryonic development [GO:0043009] Sources: GOC:cls, GOC:dgh, GOC:dph, GOC:jid, GO_REF:0000021 Definition: The process whose specific outcome is the progression of the neural tube over time, from its formation to the mature structure. The mature structure of the neural tube exists when the tube has been segmented into the forebrain, midbrain, hindbrain and spinal cord regions. In addition neural crest has budded away from the epithelium.